2-dehydro-3-deoxy-6-phosphogalactonate aldolase activity [GO:0008674] (molecular function) Also known as: 2-dehydro-3-deoxyphosphogalactonate aldolase activity, (KDPGal)aldolase activity, 2-dehydro-3-deoxy-D-galactonate-6-phosphate D-glyceraldehyde-3-phosphate-lyase (pyruvate-forming), 2-dehydro-3-deoxy-D-galactonate-6-phosphate D-glyceraldehyde-3-phosphate-lyase activity, 2-keto-3-deoxy-6-phosphogalactonic acid aldolase activity, 2-keto-3-deoxy-6-phosphogalactonic aldolase activity, 2-oxo-3-deoxygalactonate 6-phosphate aldolase activity, 6-phospho-2-dehydro-3-deoxygalactonate aldolase activity, 6-phospho-2-keto-3-deoxygalactonate aldolase activity, phospho-2-keto-3-deoxygalactonate aldolase activity, phospho-2-keto-3-deoxygalactonic aldolase activity Definition: Catalysis of the reaction: 6-phospho-2-dehydro-3-deoxy-D-galactonate = D-glyceraldehyde 3-phosphate + pyruvate. Relationships: is a type of aldehyde-lyase activity [GO:0016832] Sources: EC:4.1.2.21, RHEA:24464